immune response in nasopharyngeal-associated lymphoid tissue [GO:0002395] (biological process) Definition: An immune response taking place in the nasopharyngeal-associated lymphoid tissue (NALT). NALT includes the tonsils and adenoids. Relationships: is a type of immune response in gut-associated lymphoid tissue [GO:0002387] Sources: GOC:jal, ISBN:0781735149 Also known as: immune response in NALT Subtypes: GO:0002400